{
  "gene_symbol": "CLASP1",
  "term_id": "GO:0040001",
  "term_label": "establishment of mitotic spindle localization",
  "gene": "UniProtKB:Q7Z460",
  "gene_name": "CLIP-associating protein 1"
}